{
  "gene": "UniProtKB:A8MSI8",
  "gene_symbol": "LYRM9",
  "term_label": "Unknown biological process",
  "term_id": "UNKNOWN:0002",
  "gene_name": "LYR motif-containing protein 9"
}